{
  "gene": "UniProtKB:P0CG38",
  "gene_name": "POTE ankyrin domain family member I",
  "term_id": "GO:0035267",
  "term_label": "NuA4 histone acetyltransferase complex",
  "gene_symbol": "POTEI"
}